{
  "gene_symbol": "RECQL5",
  "gene_name": "ATP-dependent DNA helicase Q5",
  "gene": "UniProtKB:O94762",
  "term_id": "GO:0005694",
  "term_label": "chromosome"
}